{
  "gene_symbol": "REV1",
  "term_label": "nucleus",
  "gene": "UniProtKB:Q9UBZ9",
  "gene_name": "DNA repair protein REV1",
  "term_id": "GO:0005634"
}